{
  "term_label": "plasma membrane",
  "term_id": "GO:0005886",
  "gene_name": "Choline transporter-like protein 1",
  "gene_symbol": "SLC44A1",
  "gene": "UniProtKB:Q8WWI5"
}